{
  "term_label": "phosphatidylinositol dephosphorylation",
  "gene": "UniProtKB:Q13614",
  "term_id": "GO:0046856",
  "gene_name": "Myotubularin-related protein 2",
  "gene_symbol": "MTMR2"
}